{
  "gene_symbol": "RNF152",
  "gene": "UniProtKB:Q8N8N0",
  "term_id": "GO:0061630",
  "gene_name": "E3 ubiquitin-protein ligase RNF152",
  "term_label": "ubiquitin protein ligase activity"
}